{
  "gene": "UniProtKB:P25490",
  "term_id": "GO:0005667",
  "gene_symbol": "YY1",
  "gene_name": "Transcriptional repressor protein YY1",
  "term_label": "transcription regulator complex"
}